{
  "term_id": "GO:0043123",
  "gene_name": "Tumor necrosis factor ligand superfamily member 15",
  "gene": "UniProtKB:O95150",
  "term_label": "positive regulation of canonical NF-kappaB signal transduction",
  "gene_symbol": "TNFSF15"
}